naphthalene 1,2-dioxygenase activity [GO:0018625] (molecular function) Also known as: naphthalene dioxygenase activity, naphthalene oxygenase activity, naphthalene,NADH:oxygen oxidoreductase (1,2-hydroxylating) Definition: Catalysis of the reaction: naphthalene + NADH + H+ + O2 = (1R,2S)-1,2-dihydronaphthalene-1,2-diol + NAD+. Relationships: is a type of oxidoreductase activity, acting on paired donors, with incorporation or reduction of molecular oxygen, NAD(P)H as one donor, and incorporation of two atoms of oxygen into one donor [GO:0016708] Sources: EC:1.14.12.12